{
  "term_label": "nucleus",
  "gene": "UniProtKB:P28370",
  "gene_symbol": "SMARCA1",
  "term_id": "GO:0005634",
  "gene_name": "Probable global transcription activator SNF2L1"
}